{
  "gene_symbol": "TRAP1",
  "term_id": "GO:0006457",
  "term_label": "protein folding",
  "gene": "UniProtKB:Q12931",
  "gene_name": "Heat shock protein 75 kDa, mitochondrial"
}